{
  "gene_name": "5-hydroxytryptamine receptor 1B",
  "term_label": "neurotransmitter receptor activity",
  "gene_symbol": "HTR1B",
  "term_id": "GO:0030594",
  "gene": "UniProtKB:P28222"
}